optic nerve maturation [GO:0021632] (BP) Relationships: is a type of cranial nerve maturation [GO:0021605]; is part of optic nerve development [GO:0021554] Sources: GOC:cls, GOC:dgh, GOC:dph, GOC:jid, GO_REF:0000021 Definition: A developmental process, independent of morphogenetic (shape) change, that is required for the optic nerve to attain its fully functional state. The sensory optic nerve originates from the bipolar cells of the retina and conducts visual information to the brainstem. The optic nerve exits the back of the eye in the orbit, enters the optic canal, and enters the central nervous system at the optic chiasm (crossing) where the nerve fibers become the optic tract just prior to entering the hindbrain. Also known as: CN II maturation